positive regulation of ductus arteriosus closure [GO:1904337] (biological process) Definition: Any process that activates or increases the frequency, rate or extent of ductus arteriosus closure. Relationships: is a type of regulation of ductus arteriosus closure [GO:1904335]; is a type of positive regulation of artery morphogenesis [GO:1905653]; positively regulates ductus arteriosus closure [GO:0097070] Also known as: up regulation of ductus arteriosus closure, up-regulation of ductus arteriosus closure, upregulation of ductus arteriosus closure, activation of ductus arteriosus closure References: PMID:16303610 Sources: GOC:TermGenie, GO_REF:0000058